regulation of B cell receptor signaling pathway [GO:0050855] (biological process) Definition: Any process that modulates the frequency, rate or extent of signaling pathways initiated by the cross-linking of an antigen receptor on a B cell. Subtypes: negative regulation of B cell receptor signaling pathway [GO:0050859], positive regulation of B cell receptor signaling pathway [GO:0050861] Also known as: regulation of B cell receptor signalling pathway, regulation of B lymphocyte receptor signaling pathway, regulation of B lymphocyte receptor signalling pathway, regulation of B-cell receptor signaling pathway, regulation of B-cell receptor signalling pathway, regulation of B-lymphocyte receptor signaling pathway, regulation of B-lymphocyte receptor signalling pathway Relationships: is a type of regulation of antigen receptor-mediated signaling pathway [GO:0050854]; regulates B cell receptor signaling pathway [GO:0050853] Sources: GOC:ai